{
  "gene_symbol": "PLEKHJ1",
  "term_id": "GO:0005802",
  "term_label": "trans-Golgi network",
  "gene_name": "Pleckstrin homology domain-containing family J member 1",
  "gene": "UniProtKB:Q9NW61"
}